sarcomere organization [GO:0045214] (biological process) Regulation: regulated by regulation of sarcomere organization [GO:0060297]; RO_0002213 by positive regulation of sarcomere organization [GO:0060298]; negatively regulated by negative regulation of sarcomere organization [GO:0060299] Also known as: sarcomere alignment, sarcomere organisation Definition: The myofibril assembly process that results in the organization of muscle actomyosin into sarcomeres. The sarcomere is the repeating unit of a myofibril in a muscle cell, composed of an array of overlapping thick and thin filaments between two adjacent Z discs. Relationships: is a type of actomyosin structure organization [GO:0031032]; is part of myofibril assembly [GO:0030239] Sources: GOC:bf